negative regulation of protein desumoylation [GO:0060190] (BP) Definition: Any process that decreases the frequency, rate or extent of protein desumoylation. Protein desumoylation is the process in which a SUMO protein (small ubiquitin-related modifier) is cleaved from its target protein. Relationships: is a type of regulation of protein desumoylation [GO:0060188]; is a type of negative regulation of protein modification by small protein conjugation or removal [GO:1903321]; negatively regulates protein desumoylation [GO:0016926] Sources: GOC:dph, GOC:tb